{
  "term_id": "GO:0005886",
  "gene_name": "ADP-ribosylation factor-like protein 17 C-terminal domain-containing protein",
  "gene_symbol": "LOC107984156",
  "term_label": "plasma membrane",
  "gene": "UniProtKB:A0A0G2JMH3"
}